{
  "gene": "UniProtKB:Q9Y6W8",
  "gene_symbol": "ICOS",
  "term_id": "GO:0002517",
  "term_label": "T cell tolerance induction",
  "gene_name": "Inducible T-cell costimulator"
}